{
  "gene": "UniProtKB:O95453",
  "term_id": "GO:0000175",
  "gene_name": "Poly(A)-specific ribonuclease PARN",
  "term_label": "3'-5'-RNA exonuclease activity",
  "gene_symbol": "PARN"
}